{
  "term_id": "GO:0006672",
  "term_label": "ceramide metabolic process",
  "gene_name": "Phospholipase A2 group XV",
  "gene": "UniProtKB:Q8NCC3",
  "gene_symbol": "PLA2G15"
}